regulation of mesenchymal cell proliferation involved in ureter development [GO:0072199] (biological process) Also known as: regulation of ureter mesenchymal cell proliferation, regulation of ureteral mesenchymal cell proliferation Definition: Any process that modulates the frequency, rate or extent of mesenchymal cell proliferation that contributes to the progression of the ureter gland over time. A mesenchymal cell is a cell that normally gives rise to other cells that are organized as three-dimensional masses, rather than sheets. Relationships: is a type of regulation of mesenchymal cell proliferation [GO:0010464]; regulates GO:0072198 Subtypes: GO:0072200, GO:2000729 Sources: GOC:mtg_kidney_jan10